mitotic spindle midzone [GO:1990023] (cellular component) Sources: GOC:mtg_cell_cycle, GOC:vw Relationships: is a type of GO:0051233; is part of GO:0072686 Definition: The area in the center of the anaphase spindle consisting of microtubules, microtubule bundling factors and kinesin motors where the spindle microtubules from opposite poles overlap in an antiparallel manner.